{
  "gene": "UniProtKB:Q96SQ9",
  "gene_symbol": "CYP2S1",
  "term_label": "epoxygenase P450 pathway",
  "gene_name": "Cytochrome P450 2S1",
  "term_id": "GO:0019373"
}